{
  "term_label": "E-box binding",
  "gene": "UniProtKB:Q9Y4Z2",
  "gene_symbol": "NEUROG3",
  "term_id": "GO:0070888",
  "gene_name": "Neurogenin-3"
}